{
  "term_label": "diphosphoinositol polyphosphate metabolic process",
  "term_id": "GO:0071543",
  "gene_name": "Diphosphoinositol polyphosphate phosphohydrolase NUDT4B",
  "gene": "UniProtKB:A0A024RBG1",
  "gene_symbol": "NUDT4B"
}